{
  "gene_symbol": "ATAD1",
  "gene": "UniProtKB:Q8NBU5",
  "term_id": "GO:0005741",
  "term_label": "mitochondrial outer membrane",
  "gene_name": "Outer mitochondrial transmembrane helix translocase"
}